porphyrin-containing compound catabolic process [GO:0006787] (biological process) Also known as: porphyrin breakdown, porphyrin catabolic process, porphyrin catabolism, porphyrin degradation Definition: The chemical reactions and pathways resulting in the breakdown of any member of a large group of derivatives or analogs of porphyrin. Porphyrin consists of a ring of four pyrrole nuclei linked each to the next at their alpha positions through a methine group. Subtypes: bilirubin conjugation [GO:0006789], chlorophyll catabolic process [GO:0015996], heme catabolic process [GO:0042167] Sources: GOC:jl, ISBN:0198506732 Relationships: is a type of porphyrin-containing compound metabolic process [GO:0006778]; is_a tetrapyrrole catabolic process [GO:0033015]